{
  "term_label": "Unknown biological process",
  "gene_symbol": "PNKD",
  "gene_name": "Probable hydrolase PNKD",
  "gene": "UniProtKB:Q8N490",
  "term_id": "UNKNOWN:0002"
}